{
  "gene_name": "Potassium voltage-gated channel subfamily KQT member 5",
  "gene": "UniProtKB:Q9NR82",
  "gene_symbol": "KCNQ5",
  "term_id": "GO:0008076",
  "term_label": "voltage-gated potassium channel complex"
}